{
  "gene_name": "Forkhead box protein F1",
  "term_id": "GO:0006357",
  "term_label": "regulation of transcription by RNA polymerase II",
  "gene": "UniProtKB:Q12946",
  "gene_symbol": "FOXF1"
}